{
  "gene_symbol": "SPIN4",
  "gene_name": "Spindlin-4",
  "term_label": "Unknown molecular function",
  "term_id": "UNKNOWN:0001",
  "gene": "UniProtKB:Q56A73"
}